{
  "term_id": "UNKNOWN:0001",
  "term_label": "Unknown molecular function",
  "gene_symbol": "BABAM1",
  "gene": "UniProtKB:Q9NWV8",
  "gene_name": "BRISC and BRCA1-A complex member 1"
}